preblastoderm mitotic cell cycle [GO:0035185] (biological process) Sources: ISBN:0879694238 Relationships: is a type of cell cycle comprising mitosis without cytokinesis [GO:0033301]; is a type of mitotic cell cycle, embryonic [GO:0045448] Definition: The first nine mitotic division cycles of the insect embryo, during which the dividing nuclei lie deep in the interior of the egg and divide nearly synchronously. This is the first phase of the syncytial period where nuclei divide in a common cytoplasm without cytokinesis. Regulation: regulated by GO:0007347; negatively regulated by negative regulation of preblastoderm mitotic cell cycle [GO:0046001]; positively regulated by positive regulation of preblastoderm mitotic cell cycle [GO:0046002]